{
  "gene": "UniProtKB:Q9P2W3",
  "term_label": "G-protein beta-subunit binding",
  "gene_name": "Guanine nucleotide-binding protein G(I)_G(S)_G(O) subunit gamma-13",
  "term_id": "GO:0031681",
  "gene_symbol": "GNG13"
}